{
  "gene": "UniProtKB:Q969E3",
  "gene_symbol": "UCN3",
  "term_id": "GO:0009755",
  "gene_name": "Urocortin-3",
  "term_label": "hormone-mediated signaling pathway"
}